{
  "term_label": "positive regulation of nuclear cell cycle DNA replication",
  "gene_name": "Protein DBF4 homolog A",
  "term_id": "GO:0010571",
  "gene_symbol": "DBF4",
  "gene": "UniProtKB:Q9UBU7"
}